{
  "gene_symbol": "FZD10",
  "term_label": "extracellular space",
  "term_id": "GO:0005615",
  "gene": "UniProtKB:Q9ULW2",
  "gene_name": "Frizzled-10"
}